{
  "term_id": "GO:0051480",
  "gene": "UniProtKB:Q9UBN4",
  "gene_name": "Short transient receptor potential channel 4",
  "term_label": "regulation of cytosolic calcium ion concentration",
  "gene_symbol": "TRPC4"
}